chemokine (C-C motif) ligand 7 binding [GO:0035717] (molecular function) Sources: GOC:BHF Definition: Binding to chemokine (C-C motif) ligand 7. Also known as: CCL7 binding Relationships: is a type of GO:0019957